{
  "term_id": "GO:0032811",
  "gene_name": "Corticoliberin",
  "gene_symbol": "CRH",
  "term_label": "negative regulation of epinephrine secretion",
  "gene": "UniProtKB:P06850"
}